{
  "gene_name": "SID1 transmembrane family member 2",
  "gene_symbol": "SIDT2",
  "term_label": "RNA transport",
  "term_id": "GO:0050658",
  "gene": "UniProtKB:Q8NBJ9"
}